{
  "term_label": "epithelial cilium movement involved in extracellular fluid movement",
  "gene_name": "Sperm-associated antigen 6",
  "gene_symbol": "SPAG6",
  "gene": "UniProtKB:O75602",
  "term_id": "GO:0003351"
}